organophosphate biosynthetic process [GO:0090407] (biological process) Sources: GOC:chem_mtg Subtypes: phospholipid biosynthetic process [GO:0008654], GO:0009229, molybdopterin cofactor biosynthetic process [GO:0032324], inositol phosphate biosynthetic process [GO:0032958], phosphagen biosynthetic process [GO:0042396], pyridoxal phosphate biosynthetic process [GO:0042823], GO:0046166, glycerol-3-phosphate biosynthetic process [GO:0046167], deoxyribose phosphate biosynthetic process [GO:0046385], ribose phosphate biosynthetic process [GO:0046390], carbamoyl phosphate biosynthetic process [GO:0070409], GO:0140380, GO:1901159, nucleoside phosphate biosynthetic process [GO:1901293], cyclic 2,3-bisphospho-D-glycerate biosynthetic process [GO:1901369], D-glycero-D-manno-heptose 7-phosphate biosynthetic process [GO:2001061], methanopterin-containing compound biosynthetic process [GO:2001116], coenzyme gamma-F420-2 biosynthetic process [GO:2001121] Definition: The chemical reactions and pathways resulting in the biosynthesis of deoxyribose phosphate, the phosphorylated sugar 2-deoxy-erythro-pentose. Relationships: is a type of biosynthetic process [GO:0009058]; is_a organophosphate metabolic process [GO:0019637]